{
  "gene_name": "Beta-actin-like protein 2",
  "gene": "UniProtKB:Q562R1",
  "term_label": "glutamatergic synapse",
  "term_id": "GO:0098978",
  "gene_symbol": "ACTBL2"
}